{
  "gene_symbol": "TADA2B",
  "gene": "UniProtKB:Q86TJ2",
  "term_id": "GO:0003682",
  "gene_name": "Transcriptional adapter 2-beta",
  "term_label": "chromatin binding"
}